{
  "gene_symbol": "DENND2D",
  "gene_name": "DENN domain-containing protein 2D",
  "gene": "UniProtKB:Q9H6A0",
  "term_id": "UNKNOWN:0002",
  "term_label": "Unknown biological process"
}